{
  "gene": "UniProtKB:Q9UBS4",
  "gene_symbol": "DNAJB11",
  "gene_name": "DnaJ homolog subfamily B member 11",
  "term_label": "protein maturation",
  "term_id": "GO:0051604"
}